{
  "term_id": "GO:0000915",
  "gene_name": "Rhotekin",
  "gene": "UniProtKB:Q9BST9",
  "term_label": "actomyosin contractile ring assembly",
  "gene_symbol": "RTKN"
}